{
  "term_label": "regulation of transcription by RNA polymerase II",
  "gene": "UniProtKB:P17021",
  "gene_symbol": "ZNF17",
  "gene_name": "Zinc finger protein 17",
  "term_id": "GO:0006357"
}